suspensor development [GO:0010098] (biological process) Relationships: is_a anatomical structure development [GO:0048856] Sources: GOC:tb, ISBN:0471245208 Definition: The process whose specific outcome is the progression of the suspensor over time, from its formation to the mature structure. The suspensor is the extension at the base of the embryo that anchors the embryo in the embryo sac and pushes it into the endosperm.